{
  "term_id": "UNKNOWN:0002",
  "term_label": "Unknown biological process",
  "gene": "UniProtKB:Q8WTU2",
  "gene_symbol": "SSC4D",
  "gene_name": "Scavenger receptor cysteine-rich domain-containing group B protein"
}